{
  "gene_name": "N-cym protein",
  "gene": "UniProtKB:P40205",
  "term_label": "Unknown biological process",
  "term_id": "UNKNOWN:0002",
  "gene_symbol": "MYCNOS"
}